vindoline biosynthetic process [GO:1900985] (biological process) Relationships: is a type of terpenoid indole alkaloid biosynthetic process [GO:0009709]; is a type of tertiary alcohol biosynthetic process [GO:1902645] Also known as: vindoline anabolism, vindoline biosynthesis, vindoline formation, vindoline synthesis References: PMID:12228585 Sources: GOC:TermGenie, GOC:yaf Definition: The chemical reactions and pathways resulting in the formation of vindoline.